dihydrosphingosine-1-phosphate phosphatase activity [GO:0070780] (molecular function) References: PMID:12815058 Sources: GOC:pde Also known as: dihydrosphingosine-1-phosphate phosphohydrolase activity, sphinganine-1-phosphate phosphatase activity Definition: Catalysis of the reaction: dihydrosphingosine 1-phosphate + H2O = dihydrosphingosine + phosphate. Relationships: is a type of phosphatase activity [GO:0016791]